{
  "gene_symbol": "MLNR",
  "term_id": "GO:0005886",
  "gene": "UniProtKB:O43193",
  "term_label": "plasma membrane",
  "gene_name": "Motilin receptor"
}